{
  "term_id": "GO:0090734",
  "gene": "UniProtKB:Q6PCD5",
  "gene_symbol": "RFWD3",
  "gene_name": "E3 ubiquitin-protein ligase RFWD3",
  "term_label": "site of DNA damage"
}